mycotoxin catabolic process [GO:0043387] (BP) Definition: The chemical reactions and pathways resulting in the breakdown of a mycotoxin, any poisonous substance produced by a fungus. Subtypes: aflatoxin catabolic process [GO:0046223], gliotoxin catabolic process [GO:2001309] Sources: GOC:jl Also known as: mycotoxin breakdown, mycotoxin catabolism, mycotoxin degradation Relationships: is a type of GO:0009407; is a type of mycotoxin metabolic process [GO:0043385]